muscle attachment [GO:0016203] (biological process) Relationships: is a type of GO:0032501; is part of skeletal muscle organ development [GO:0060538] Sources: GOC:isa_complete, GOC:sart Definition: The developmental process in which a skeletal muscle attaches to its target (such as bone or body wall).